{
  "term_id": "GO:0015721",
  "term_label": "bile acid and bile salt transport",
  "gene_name": "Sodium_bile acid cotransporter 4",
  "gene": "UniProtKB:Q96EP9",
  "gene_symbol": "SLC10A4"
}